{
  "gene_name": "Lysyl oxidase homolog 3",
  "gene": "UniProtKB:P58215",
  "term_id": "GO:0005615",
  "gene_symbol": "LOXL3",
  "term_label": "extracellular space"
}